meiotic anaphase I [GO:0007133] (biological process) Relationships: is a type of GO:0098764; is part of anaphase [GO:0051322]; is part of GO:0051327 Note: Note that this term should not be used for direct annotation. If you are trying to make an annotation to x phase, it is likely that the correct annotation is 'regulation of x/y phase transition' or to a process which occurs during the reported phase (i.e mitotic DNA replication for mitotic S-phase). To capture the phase when a specific location or process is observed, the phase term can be used in an annotation extension (PMID:24885854) applied to a cellular component term (with the relation exists_during) or a biological process term (with the relation happens_during). Definition: The cell cycle phase during which chromosomes separate and migrate towards the poles of the spindle the as part of meiosis I. Sources: GOC:mtg_cell_cycle